{
  "gene_name": "CB1 cannabinoid receptor-interacting protein 1",
  "term_label": "Unknown biological process",
  "gene_symbol": "CNRIP1",
  "gene": "UniProtKB:Q96F85",
  "term_id": "UNKNOWN:0002"
}